complement-mediated synapse pruning [GO:0150062] (biological process) Definition: Synaptic pruning mediated by complement system signaling. References: PMID:18083105, PMID:22632727, PMID:29844190 Sources: GOC:aruk, GOC:bc Relationships: is a type of synapse pruning [GO:0098883] Also known as: synapse clearance, synapse disassembly, synapse elimination, synapse removal, complement-dependent synapse pruning